{
  "term_id": "GO:0031210",
  "gene_name": "Choline-phosphate cytidylyltransferase A",
  "term_label": "phosphatidylcholine binding",
  "gene": "UniProtKB:P49585",
  "gene_symbol": "PCYT1A"
}